{
  "gene": "UniProtKB:Q9NXA8",
  "term_label": "mitochondrial matrix",
  "gene_name": "NAD-dependent protein deacylase sirtuin-5, mitochondrial",
  "gene_symbol": "SIRT5",
  "term_id": "GO:0005759"
}